{
  "gene": "UniProtKB:P04259",
  "gene_name": "Keratin, type II cytoskeletal 6B",
  "term_label": "intermediate filament organization",
  "term_id": "GO:0045109",
  "gene_symbol": "KRT6B"
}